{
  "gene_symbol": "CAV1",
  "gene_name": "Caveolin-1",
  "gene": "UniProtKB:Q03135",
  "term_id": "GO:0005794",
  "term_label": "Golgi apparatus"
}